{
  "term_label": "protein disulfide isomerase activity",
  "term_id": "GO:0003756",
  "gene": "UniProtKB:Q6ZRP7",
  "gene_name": "Sulfhydryl oxidase 2",
  "gene_symbol": "QSOX2"
}